photosynthetic electron transport in photosystem I [GO:0009773] (biological process) Sources: GOC:jid, ISBN:0716731363, ISBN:0816017360 Relationships: is a type of GO:0009767 Definition: A photosynthetic electron transport chain in which electrons move from the primary electron acceptor (Quinone, X) through a chain of electron transport molecules in the thylakoid membrane until they reach ferredoxin which passes the electron to the ultimate electron acceptor; NADP.